neurotrophin receptor activity [GO:0005030] (molecular function) Relationships: is a type of signaling receptor activity [GO:0038023]; is part of neurotrophin signaling pathway [GO:0038179]; has part neurotrophin binding [GO:0043121] Subtypes: nerve growth factor receptor activity [GO:0010465], brain-derived neurotrophic factor receptor activity [GO:0060175] Definition: Combining with a neurotrophin, any of a family of growth factors that prevent apoptosis in neurons and promote nerve growth, and transmitting the signal to initiate a change in cell activity. Sources: GOC:jl, GOC:signaling